{
  "gene_symbol": "PTH2R",
  "gene": "UniProtKB:P49190",
  "term_id": "GO:0008528",
  "gene_name": "Parathyroid hormone 2 receptor",
  "term_label": "G protein-coupled peptide receptor activity"
}